negative regulation of mitophagy [GO:1901525] (biological process) Relationships: is a type of negative regulation of macroautophagy [GO:0016242]; is a type of GO:1901524; is a type of GO:1903147; negatively regulates mitophagy [GO:0000423] Also known as: down regulation of macromitophagy, down-regulation of macromitophagy, downregulation of macromitophagy, negative regulation of macromitophagy, inhibition of macromitophagy Subtypes: negative regulation of type 2 mitophagy [GO:1905090] Definition: Any process that stops, prevents or reduces the frequency, rate or extent of mitophagy. Sources: GOC:TermGenie